{
  "term_label": "cysteine-type deubiquitinase activity",
  "gene_symbol": "USP17L11",
  "gene_name": "Ubiquitin carboxyl-terminal hydrolase 17-like protein 11",
  "term_id": "GO:0004843",
  "gene": "UniProtKB:C9JVI0"
}